{
  "gene_name": "Actin, cytoplasmic 1",
  "term_id": "GO:0045202",
  "gene_symbol": "ACTB",
  "term_label": "synapse",
  "gene": "UniProtKB:P60709"
}